{
  "gene_name": "Zinc finger protein 668",
  "term_label": "transcription cis-regulatory region binding",
  "term_id": "GO:0000976",
  "gene_symbol": "ZNF668",
  "gene": "UniProtKB:Q96K58"
}